{
  "term_id": "GO:0032977",
  "gene_symbol": "EMC8",
  "gene_name": "ER membrane protein complex subunit 8",
  "term_label": "membrane insertase activity",
  "gene": "UniProtKB:O43402"
}